{
  "term_id": "GO:0005737",
  "gene_name": "Serine_threonine-protein phosphatase 2B catalytic subunit gamma isoform",
  "term_label": "cytoplasm",
  "gene_symbol": "PPP3CC",
  "gene": "UniProtKB:P48454"
}